{
  "gene": "UniProtKB:O00230",
  "term_id": "GO:0005184",
  "term_label": "neuropeptide hormone activity",
  "gene_name": "Cortistatin",
  "gene_symbol": "CORT"
}